{
  "term_label": "plasma membrane",
  "gene_name": "Spectrin beta chain, non-erythrocytic 4",
  "term_id": "GO:0005886",
  "gene": "UniProtKB:Q9H254",
  "gene_symbol": "SPTBN4"
}